{
  "gene": "UniProtKB:Q96PU4",
  "gene_name": "E3 ubiquitin-protein ligase UHRF2",
  "term_id": "GO:0061630",
  "term_label": "ubiquitin protein ligase activity",
  "gene_symbol": "UHRF2"
}